{
  "term_label": "Unknown molecular function",
  "term_id": "UNKNOWN:0001",
  "gene_name": "WD repeat-containing protein 25",
  "gene_symbol": "WDR25",
  "gene": "UniProtKB:Q64LD2"
}